{
  "term_label": "bile acid biosynthetic process",
  "gene_name": "Cytochrome P450 7A1",
  "gene": "UniProtKB:P22680",
  "term_id": "GO:0006699",
  "gene_symbol": "CYP7A1"
}